{
  "gene_symbol": "GBA2",
  "term_label": "central nervous system development",
  "gene": "UniProtKB:Q9HCG7",
  "gene_name": "Non-lysosomal glucosylceramidase",
  "term_id": "GO:0007417"
}